{
  "gene_symbol": "PGRMC1",
  "gene_name": "Membrane-associated progesterone receptor component 1",
  "term_id": "GO:0005783",
  "gene": "UniProtKB:O00264",
  "term_label": "endoplasmic reticulum"
}